{
  "gene_symbol": "ISL1",
  "term_label": "cis-regulatory region sequence-specific DNA binding",
  "gene_name": "Insulin gene enhancer protein ISL-1",
  "gene": "UniProtKB:P61371",
  "term_id": "GO:0000987"
}